L-Ala-D/L-Glu epimerase activity [GO:0103031] (MF) Definition: Catalysis of the reaction:L-alanyl-L-glutamate = L-alanyl-D-glutamate. Sources: RHEA:28394 Relationships: is a type of racemase and epimerase activity, acting on amino acids and derivatives [GO:0016855]